{
  "gene": "UniProtKB:P07333",
  "term_label": "regulation of MAPK cascade",
  "term_id": "GO:0043408",
  "gene_name": "Macrophage colony-stimulating factor 1 receptor",
  "gene_symbol": "CSF1R"
}